{
  "gene_name": "Bis(5'-nucleosyl)-tetraphosphatase [asymmetrical]",
  "term_label": "bis(5'-nucleosyl)-tetraphosphatase (asymmetrical) activity",
  "term_id": "GO:0004081",
  "gene_symbol": "NUDT2",
  "gene": "UniProtKB:P50583"
}